{
  "term_label": "Unknown biological process",
  "term_id": "UNKNOWN:0002",
  "gene_symbol": "FBXO15",
  "gene_name": "F-box only protein 15",
  "gene": "UniProtKB:Q8NCQ5"
}